{
  "gene": "UniProtKB:P0CF51",
  "gene_name": "T cell receptor gamma constant 1",
  "term_label": "Unknown molecular function",
  "gene_symbol": "TRGC1",
  "term_id": "UNKNOWN:0001"
}